activation of protein kinase A activity [GO:0034199] (biological process) Also known as: protein kinase A activation Definition: Any process that initiates the activity of the inactive enzyme protein kinase A. Relationships: is a type of activation of protein kinase activity [GO:0032147] Sources: GOC:pde